{
  "term_id": "UNKNOWN:0001",
  "gene_symbol": "METTL27",
  "gene": "UniProtKB:Q8N6F8",
  "gene_name": "Methyltransferase-like protein 27",
  "term_label": "Unknown molecular function"
}